plant gross anatomical part developmental process [GO:0160109] (biological process) Relationships: is a type of GO:0032502 Also known as: plant development Sources: GOC:pg Definition: Any developmental process whose specific outcome is the progression of a gross anatomical part of a plant from an initial immature state, to a later, more mature state.